{
  "gene_name": "Zinc finger protein 43",
  "term_label": "transcription cis-regulatory region binding",
  "term_id": "GO:0000976",
  "gene": "UniProtKB:P17038",
  "gene_symbol": "ZNF43"
}